{
  "gene_name": "Acyl-protein thioesterase 2",
  "term_label": "palmitoyl-(protein) hydrolase activity",
  "gene_symbol": "LYPLA2",
  "term_id": "GO:0008474",
  "gene": "UniProtKB:O95372"
}